positive regulation of nucleocytoplasmic transport [GO:0046824] (biological process) Subtypes: GO:0042307, positive regulation of protein export from nucleus [GO:0046827], GO:0046830, positive regulation of RNA export from nucleus [GO:0046833], positive regulation of ribosomal subunit export from nucleus [GO:2000202] Also known as: up regulation of nucleocytoplasmic transport, up-regulation of nucleocytoplasmic transport, upregulation of nucleocytoplasmic transport, activation of nucleocytoplasmic transport, stimulation of nucleocytoplasmic transport Definition: Any process that activates or increases the frequency, rate or extent of the directed movement of substances between the nucleus and the cytoplasm. Sources: GOC:bf Relationships: is a type of positive regulation of intracellular transport [GO:0032388]; is_a regulation of nucleocytoplasmic transport [GO:0046822]; positively regulates nucleocytoplasmic transport [GO:0006913]